{
  "gene_name": "Semaphorin-4D",
  "gene": "UniProtKB:Q92854",
  "gene_symbol": "SEMA4D",
  "term_id": "GO:0001755",
  "term_label": "neural crest cell migration"
}